negative regulation of opioid receptor signaling pathway [GO:2000475] (biological process) Subtypes: negative regulation of adenylate cyclase-inhibiting opioid receptor signaling pathway [GO:1900730] Definition: Any process that stops, prevents or reduces the frequency, rate or extent of opioid receptor signaling pathway. Sources: GOC:obol Also known as: negative regulation of opioid receptor signalling pathway Relationships: is a type of negative regulation of G protein-coupled receptor signaling pathway [GO:0045744]; is a type of regulation of opioid receptor signaling pathway [GO:2000474]; negatively regulates G protein-coupled opioid receptor signaling pathway [GO:0038003]